{
  "term_label": "plasma membrane",
  "term_id": "GO:0005886",
  "gene_name": "Serine_threonine-protein kinase receptor R3",
  "gene_symbol": "ACVRL1",
  "gene": "UniProtKB:P37023"
}